{
  "gene_name": "Putative RNA polymerase II subunit B1 CTD phosphatase RPAP2",
  "term_label": "Unknown biological process",
  "gene_symbol": "RPAP2",
  "gene": "UniProtKB:Q8IXW5",
  "term_id": "UNKNOWN:0002"
}